{
  "term_id": "GO:0019814",
  "gene": "UniProtKB:A0A075B6I6",
  "gene_name": "Probable non-functional immunoglobulin lambda variable 1-50",
  "gene_symbol": "IGLV1-50",
  "term_label": "immunoglobulin complex"
}